{
  "term_id": "GO:0001817",
  "term_label": "regulation of cytokine production",
  "gene": "UniProtKB:A0A1B0GVX0",
  "gene_name": "LITAF domain-containing protein",
  "gene_symbol": "LITAFD"
}